tongue development [GO:0043586] (biological process) Sources: GOC:jl, UBERON:0001723 Relationships: is a type of GO:0007423 Definition: The process whose specific outcome is the progression of the tongue over time, from its formation to the mature structure. The tongue is the movable, muscular organ on the floor of the mouth of most vertebrates, in many other mammals is the principal organ of taste, aids in the prehension of food, in swallowing, and in modifying the voice as in speech. Also known as: glossa development, lingua development